positive regulation of protein localization to nucleus [GO:1900182] (biological process) Subtypes: GO:0042307, positive regulation of protein localization to nucleolus [GO:1904751], positive regulation of protein localization to Cajal body [GO:1904871] Relationships: is a type of regulation of protein localization to nucleus [GO:1900180]; is a type of positive regulation of protein localization [GO:1903829]; positively regulates protein localization to nucleus [GO:0034504] Sources: GOC:TermGenie Also known as: activation of protein localization in nucleus, positive regulation of protein localisation to nucleus, positive regulation of protein localization in cell nucleus, positive regulation of protein localization in nucleus, up regulation of protein localisation to nucleus, up regulation of protein localization in cell nucleus, up regulation of protein localization in nucleus, up regulation of protein localization to nucleus, up-regulation of protein localisation to nucleus, up-regulation of protein localization in cell nucleus, up-regulation of protein localization in nucleus, up-regulation of protein localization to nucleus, upregulation of protein localisation to nucleus, upregulation of protein localization in cell nucleus, upregulation of protein localization in nucleus, upregulation of protein localization to nucleus, activation of protein localisation to nucleus, activation of protein localization in cell nucleus, activation of protein localization to nucleus Definition: Any process that activates or increases the frequency, rate or extent of protein localization to nucleus.